{
  "term_id": "UNKNOWN:0001",
  "gene_symbol": "ATAD3A",
  "gene_name": "ATPase family AAA domain-containing protein 3A",
  "gene": "UniProtKB:Q9NVI7",
  "term_label": "Unknown molecular function"
}